determination of stomach left/right asymmetry [GO:0071909] (biological process) Relationships: is a type of determination of digestive tract left/right asymmetry [GO:0071907]; is part of GO:0062094 Definition: Determination of the asymmetric location of the stomach with respect to the left and right halves of the organism. Sources: GOC:cvs